glycolaldehyde dehydrogenase (NAD+) activity [GO:0050569] (molecular function) Relationships: is_a aldehyde dehydrogenase (NAD+) activity [GO:0004029] Sources: RHEA:20001 Also known as: glycol aldehyde dehydrogenase activity, glycolaldehyde:NAD+ oxidoreductase activity Definition: Catalysis of the reaction: glycolaldehyde + H2O + NAD+ = glycolate + 2 H+ + NADH.